{
  "term_label": "nucleus",
  "term_id": "GO:0005634",
  "gene_symbol": "USP17L13",
  "gene_name": "Ubiquitin carboxyl-terminal hydrolase 17-like protein 13",
  "gene": "UniProtKB:C9JLJ4"
}